{
  "gene": "UniProtKB:Q15546",
  "gene_symbol": "MMD",
  "gene_name": "Monocyte to macrophage differentiation factor",
  "term_label": "Unknown cellular component",
  "term_id": "UNKNOWN:0003"
}